keratinocyte differentiation [GO:0030216] (biological process) Relationships: is a type of epidermal cell differentiation [GO:0009913]; is part of skin development [GO:0043588] Regulation: regulated by regulation of keratinocyte differentiation [GO:0045616]; negatively regulated by negative regulation of keratinocyte differentiation [GO:0045617]; positively regulated by positive regulation of keratinocyte differentiation [GO:0045618] Also known as: keratinocyte cell differentiation Subtypes: limb spinous cell differentiation [GO:0060890], GO:0060891 Definition: The process in which a relatively unspecialized cell acquires specialized features of a keratinocyte. Sources: GOC:dph, GOC:mah, GOC:sdb_2009, GOC:tb